{
  "gene": "UniProtKB:O95295",
  "gene_symbol": "SNAPIN",
  "term_id": "GO:0008021",
  "gene_name": "SNARE-associated protein Snapin",
  "term_label": "synaptic vesicle"
}